Golgi to transport vesicle transport [GO:0055108] (biological process) Definition: The directed movement of proteins from the Golgi to a transport vesicle. Continuously secreted proteins are sorted into transport vesicles that fuse with the plasma membrane, releasing their contents by exocytosis. Sources: GOC:jid Relationships: is a type of intracellular transport [GO:0046907]; is part of Golgi vesicle transport [GO:0048193]